{
  "term_id": "GO:0005737",
  "gene_name": "PX domain-containing protein kinase-like protein",
  "gene_symbol": "PXK",
  "gene": "UniProtKB:Q7Z7A4",
  "term_label": "cytoplasm"
}